{
  "gene_name": "Shadow of prion protein",
  "gene_symbol": "SPRN",
  "term_label": "nucleus",
  "gene": "UniProtKB:Q5BIV9",
  "term_id": "GO:0005634"
}